protein K6-linked ubiquitination [GO:0085020] (biological process) Relationships: is a type of protein polyubiquitination [GO:0000209] Sources: GOC:sp Also known as: protein K6-linked polyubiquitination Definition: A protein ubiquitination process in which a polymer of ubiquitin, formed by linkages between lysine residues at position 6 of the ubiquitin monomers, is added to a protein. K6-linked ubiquitination is involved in DNA repair.